{
  "term_label": "Unknown biological process",
  "term_id": "UNKNOWN:0002",
  "gene_symbol": "MFSD9",
  "gene": "UniProtKB:Q8NBP5",
  "gene_name": "Major facilitator superfamily domain-containing protein 9"
}